heparan sulfate 2-sulfotransferase activity [GO:0004394] (molecular function) Definition: Catalysis of the reaction: 3'-phosphoadenosine 5'-phosphosulfate + heparan sulfate = adenosine 3',5'-bisphosphate + heparan sulfate 2-O-sulfate; results in 2-O-sulfation of iduronic acid residues in heparan sulfate. Also known as: heparan sulfate 2-O-sulfotransferase activity, heparan-sulfate 2-O-sulphotransferase activity, heparin 2-sulfotransferase activity, heparin-sulphate 2-sulphotransferase activity Relationships: is a type of heparan sulfate sulfotransferase activity [GO:0034483] References: PMID:9153262